{
  "gene": "UniProtKB:A0A1W2PQC6",
  "term_label": "mRNA cleavage and polyadenylation specificity factor complex",
  "gene_symbol": "SSU72L4",
  "gene_name": "RNA polymerase II subunit A C-terminal domain phosphatase SSU72 like protein 4",
  "term_id": "GO:0005847"
}